post-embryonic body morphogenesis [GO:0040032] (biological process) Definition: The process in which the anatomical structures of the post-embryonic soma are generated and organized. Note: Note that this term was 'body morphogenesis (sensu Nematoda)'. Sources: GOC:ems, ISBN:0140512888 Relationships: is a type of post-embryonic animal morphogenesis [GO:0009886]; is a type of GO:0010171